{
  "gene": "UniProtKB:P17066",
  "term_id": "GO:0042026",
  "gene_symbol": "HSPA6",
  "term_label": "protein refolding",
  "gene_name": "Heat shock 70 kDa protein 6"
}